{
  "term_label": "heterotrimeric G-protein complex",
  "term_id": "GO:0005834",
  "gene_name": "Guanine nucleotide-binding protein G(o) subunit alpha",
  "gene_symbol": "GNAO1",
  "gene": "UniProtKB:P09471"
}